DNA geometric change [GO:0032392] (biological process) Definition: The process in which a transformation is induced in the geometry of a DNA double helix, resulting in a change in twist, writhe, or both, but with no change in linking number. Includes the unwinding of double-stranded DNA by helicases. Note: Note that DNA geometric change and DNA topological change (GO:0006265) are distinct, but are usually coupled in vivo. Sources: GOC:mah Relationships: is a type of DNA conformation change [GO:0071103]